regulation of response to stress [GO:0080134] (biological process) Definition: Any process that modulates the frequency, rate or extent of a response to stress. Response to stress is a change in state or activity of a cell or an organism (in terms of movement, secretion, enzyme production, gene expression, etc.) as a result of a disturbance in organismal or cellular homeostasis, usually, but not necessarily, exogenous (e.g. temperature, humidity, ionizing radiation). Sources: GOC:dhl Subtypes: regulation of vernalization response [GO:0010219], regulation of defense response [GO:0031347], regulation of response to osmotic stress [GO:0047484], GO:0080135, regulation of filamentous growth of a population of unicellular organisms in response to heat [GO:1900431], GO:1900434, GO:1902882, regulation of response to wounding [GO:1903034], GO:1903242, regulation of fear response [GO:1903365], regulation of stress response to copper ion [GO:1903853], GO:2000070 Relationships: is a type of regulation of response to stimulus [GO:0048583]; regulates response to stress [GO:0006950] Note: Note that this term is in the subset of terms that should not be used for direct gene product annotation. Instead, select a child term or, if no appropriate child term exists, please request a new term. Direct annotations to this term may be amended during annotation QC.